prothoracic disc development [GO:0035219] (biological process) Definition: Progression of the prothoracic disc over time, from its initial formation through to its metamorphosis to form the adult humerous and anterior spiracle. Relationships: is a type of imaginal disc development [GO:0007444] Sources: GOC:bf, ISBN:0879694238